{
  "gene_name": "Cancer_testis antigen family 45 member A7",
  "term_id": "UNKNOWN:0003",
  "term_label": "Unknown cellular component",
  "gene_symbol": "CT45A7",
  "gene": "UniProtKB:P0DMV0"
}